oxanine DNA N-glycosylase activity [GO:0097509] (molecular function) Relationships: is a type of deaminated base DNA N-glycosylase activity [GO:0097506] Also known as: oxanine-DNA glycosylase activity References: PMID:18789404 Sources: GOC:al Definition: DNA N-glycosylase activity acting on deaminated guanine where the resulting base (oxanine) is generated by NO- or HNO2-induced nitrosative deamination.